{
  "term_id": "GO:0005789",
  "gene_name": "Inositol 1,4,5-triphosphate receptor associated 2",
  "gene": "UniProtKB:Q12912",
  "gene_symbol": "IRAG2",
  "term_label": "endoplasmic reticulum membrane"
}